{
  "gene_name": "Solute carrier family 15 member 4",
  "term_label": "dipeptide transmembrane transporter activity",
  "gene_symbol": "SLC15A4",
  "gene": "UniProtKB:Q8N697",
  "term_id": "GO:0071916"
}